negative regulation of cellobiose catabolic process [GO:1900283] (BP) Definition: Any process that stops, prevents or reduces the frequency, rate or extent of cellobiose catabolic process. Relationships: is a type of negative regulation of catabolic process [GO:0009895]; is a type of negative regulation of carbohydrate metabolic process [GO:0045912]; is a type of regulation of cellobiose catabolic process [GO:1900282]; negatively regulates cellobiose catabolic process [GO:2000892] Sources: GOC:TermGenie, GOC:mengo_curators Also known as: down regulation of cellobiose catabolic process, down regulation of cellobiose catabolism, down-regulation of cellobiose catabolic process, down-regulation of cellobiose catabolism, downregulation of cellobiose catabolic process, downregulation of cellobiose catabolism, negative regulation of cellobiose catabolism, inhibition of cellobiose catabolic process, inhibition of cellobiose catabolism